2,3-dihydroxybenzoate--[aryl-carrier protein] ligase [GO:0008668] (molecular function) Sources: RHEA:61652 Definition: Catalysis of the reaction: 2,3-dihydroxybenzoate + ATP + holo-[ACP] = 2,3-dihydroxybenzoyl-[ACP] + AMP + diphosphate. Also known as: (2,3-dihydroxybenzoyl)adenylate synthase activity, 2,3-dihydroxybenzoate-AMP ligase activity Relationships: is a type of acid-thiol ligase activity [GO:0016878]